{
  "gene_name": "Solute carrier family 2, facilitated glucose transporter member 12",
  "gene": "UniProtKB:Q8TD20",
  "term_label": "D-glucose transmembrane transporter activity",
  "term_id": "GO:0055056",
  "gene_symbol": "SLC2A12"
}